glutamate transmembrane import into vacuole [GO:0090454] (biological process) Also known as: vacuolar glutamate import Relationships: is a type of dicarboxylic acid transport [GO:0006835]; is a type of acidic amino acid transport [GO:0015800]; is a type of amino acid transmembrane import into vacuole [GO:0032975]; is a type of nitrogen compound transport [GO:0071705]; is a type of carboxylic acid transmembrane transport [GO:1905039] Subtypes: L-glutamate transmembrane import into vacuole [GO:0090515] Definition: The directed movement of glutamate into the vacuole across the vacuolar membrane. Sources: GOC:tb